{
  "term_id": "GO:0030182",
  "gene_name": "Protein Wnt-6",
  "term_label": "neuron differentiation",
  "gene": "UniProtKB:Q9Y6F9",
  "gene_symbol": "WNT6"
}